high-affinity IgG receptor activity [GO:0019771] (molecular function) Relationships: is a type of IgG receptor activity [GO:0019770] Definition: Combining with high affinity with an immunoglobulin of an IgG isotype via the Fc region, and transmitting the signal from one side of the membrane to the other to initiate a change in cell activity. Sources: GOC:add, GOC:signaling, ISBN:0781735149 Also known as: high affinity IgG receptor activity, high affinity Fc receptor activity